{
  "gene_name": "Transcription factor ATOH7",
  "gene": "UniProtKB:Q8N100",
  "term_label": "axon development",
  "gene_symbol": "ATOH7",
  "term_id": "GO:0061564"
}